{
  "gene_name": "E3 ubiquitin-protein ligase CBL-C",
  "term_label": "ubiquitin protein ligase activity",
  "term_id": "GO:0061630",
  "gene_symbol": "CBLC",
  "gene": "UniProtKB:Q9ULV8"
}